barbed-end actin filament uncapping [GO:0051638] (biological process) Also known as: barbed end F-actin uncapping, barbed end actin filament uncapping, barbed-end F-actin uncapping, plus end F-actin uncapping, plus end actin filament uncapping, plus-end F-actin uncapping, plus-end actin filament uncapping Relationships: is a type of actin filament uncapping [GO:0051695] Sources: GOC:pf Definition: The removal of capping protein from the barbed (or plus) end of actin filaments to free the ends for addition, exchange or removal of further actin subunits.